{
  "term_id": "GO:0008202",
  "gene_name": "Cytochrome P450 3A43",
  "term_label": "steroid metabolic process",
  "gene_symbol": "CYP3A43",
  "gene": "UniProtKB:Q9HB55"
}